{
  "term_id": "GO:0003713",
  "gene_name": "Catenin beta-1",
  "gene": "UniProtKB:P35222",
  "term_label": "transcription coactivator activity",
  "gene_symbol": "CTNNB1"
}